{
  "gene_symbol": "MEI4",
  "gene_name": "Meiosis-specific protein MEI4",
  "gene": "UniProtKB:A8MW99",
  "term_id": "GO:0007129",
  "term_label": "homologous chromosome pairing at meiosis"
}